anthraniloyl-CoA monooxygenase activity [GO:0018673] (molecular function) Sources: EC:1.14.13.40 Definition: Catalysis of the reaction: 2-aminobenzoyl-CoA + 2 NADPH + 2 H+ + O2 = 2-amino-5-oxocyclohex-1-enecarboxyl-CoA + H2O + 2 NADP+. Also known as: 2-aminobenzoyl-CoA monooxygenase/reductase activity, 2-aminobenzoyl-CoA,NAD(P)H:oxygen oxidoreductase (de-aromatizing), anthraniloyl coenzyme A reductase activity Relationships: is a type of oxidoreductase activity, acting on paired donors, with incorporation or reduction of molecular oxygen, NAD(P)H as one donor, and incorporation of one atom of oxygen [GO:0016709]